{
  "term_id": "GO:0005737",
  "gene_symbol": "CRTC2",
  "gene": "UniProtKB:Q53ET0",
  "term_label": "cytoplasm",
  "gene_name": "CREB-regulated transcription coactivator 2"
}